{
  "term_label": "cell surface",
  "gene_symbol": "CEACAM20",
  "gene": "UniProtKB:Q6UY09",
  "gene_name": "Carcinoembryonic antigen-related cell adhesion molecule 20",
  "term_id": "GO:0009986"
}